{
  "gene_name": "Vacuolar protein sorting-associated protein 16 homolog",
  "term_label": "vacuole fusion, non-autophagic",
  "term_id": "GO:0042144",
  "gene_symbol": "VPS16",
  "gene": "UniProtKB:Q9H269"
}